{
  "term_label": "Unknown molecular function",
  "gene_symbol": "NKAPD1",
  "gene_name": "Uncharacterized protein NKAPD1",
  "gene": "UniProtKB:Q6ZUT1",
  "term_id": "UNKNOWN:0001"
}